{
  "gene_name": "WD repeat-containing protein 64",
  "gene": "UniProtKB:B1ANS9",
  "term_id": "UNKNOWN:0001",
  "term_label": "Unknown molecular function",
  "gene_symbol": "WDR64"
}